{
  "gene_symbol": "PLXNB3",
  "gene": "UniProtKB:Q9ULL4",
  "term_label": "semaphorin-plexin signaling pathway",
  "term_id": "GO:0071526",
  "gene_name": "Plexin-B3"
}